{
  "term_label": "Unknown biological process",
  "gene_symbol": "TMEM101",
  "term_id": "UNKNOWN:0002",
  "gene_name": "Transmembrane protein 101",
  "gene": "UniProtKB:Q96IK0"
}